{
  "term_label": "DNA-binding transcription factor activity, RNA polymerase II-specific",
  "gene_name": "Transcription factor HES-1",
  "term_id": "GO:0000981",
  "gene_symbol": "HES1",
  "gene": "UniProtKB:Q14469"
}